{
  "gene_symbol": "AUTS2",
  "term_id": "UNKNOWN:0002",
  "gene": "UniProtKB:Q8WXX7",
  "term_label": "Unknown biological process",
  "gene_name": "Autism susceptibility gene 2 protein"
}